low-density lipoprotein receptor particle metabolic process [GO:0032799] (biological process) Definition: The chemical reactions and pathways involving low-density lipoprotein receptors. Subtypes: GO:0032802 Also known as: LDL receptor metabolic process, low-density lipoprotein receptor metabolic process, low-density lipoprotein receptor metabolism Relationships: is a type of GO:0043112 Sources: GOC:vk